{
  "gene_name": "Polyhomeotic-like protein 2",
  "term_label": "nucleus",
  "gene_symbol": "PHC2",
  "term_id": "GO:0005634",
  "gene": "UniProtKB:Q8IXK0"
}